regulation of synaptic vesicle fusion to presynaptic active zone membrane [GO:0031630] (biological process) Relationships: is a type of regulation of vesicle fusion [GO:0031338]; is a type of regulation of synaptic vesicle membrane organization [GO:1901632]; regulates synaptic vesicle fusion to presynaptic active zone membrane [GO:0031629] Sources: GOC:mah Subtypes: negative regulation of synaptic vesicle fusion to presynaptic active zone membrane [GO:0031631], positive regulation of synaptic vesicle fusion to presynaptic active zone membrane [GO:0031632], GO:0150037 Also known as: regulation of synaptic vesicle fusion to pre-synaptic membrane, regulation of synaptic vesicle fusion to presynaptic membrane Definition: Any process that modulates the frequency, rate or extent of synaptic vesicle fusion to the presynaptic membrane.